cysteine transmembrane transport [GO:1903712] (biological process) References: PMID:17435223 Sources: GOC:TermGenie, GO_REF:0000069 Definition: The directed movement of cysteine across a membrane. Relationships: is a type of GO:0003333; is a type of cysteine transport [GO:0042883]; is a type of GO:1905039 Subtypes: cysteine export across plasma membrane [GO:0033228]